{
  "gene_symbol": "ADAMTSL2",
  "gene_name": "ADAMTS-like protein 2",
  "term_id": "UNKNOWN:0001",
  "term_label": "Unknown molecular function",
  "gene": "UniProtKB:Q86TH1"
}